pyrimidine ribonucleoside monophosphate metabolic process [GO:0009173] (biological process) Subtypes: pyrimidine ribonucleoside monophosphate biosynthetic process [GO:0009174], pyrimidine ribonucleoside monophosphate catabolic process [GO:0009175], CMP metabolic process [GO:0046035], TMP metabolic process [GO:0046044], UMP metabolic process [GO:0046049] Sources: GOC:go_curators, ISBN:0198506732 Relationships: is a type of GO:0009129 Also known as: pyrimidine ribonucleoside monophosphate metabolism Definition: The chemical reactions and pathways involving pyrimidine ribonucleoside monophosphate, a compound consisting of a pyrimidine base linked to a ribose sugar esterified with phosphate on the sugar.